{
  "term_id": "UNKNOWN:0003",
  "gene_name": "Putative uncharacterized protein SNHG12",
  "gene": "UniProtKB:Q9BXW3",
  "gene_symbol": "SNHG12",
  "term_label": "Unknown cellular component"
}